bilirubin transmembrane transporter activity [GO:0015127] (molecular function) Definition: Enables the transfer of bilirubin from one side of a membrane to the other. Bilirubin is a linear tetrapyrrole produced in the reticuloendothelial system from biliverdin and transported to the liver as a complex with serum albumin. In the liver, bilirubin is converted to bilirubin bisglucuronide, which is excreted in the bile. Sources: GOC:ai, ISBN:0198547684 Relationships: is a type of GO:0005310; is part of GO:0015723